{
  "term_label": "negative regulation of mitotic cell cycle",
  "gene_name": "Cyclin-dependent kinase inhibitor 1C",
  "gene_symbol": "CDKN1C",
  "term_id": "GO:0045930",
  "gene": "UniProtKB:P49918"
}